{
  "term_id": "UNKNOWN:0003",
  "gene_symbol": "SNRK",
  "term_label": "Unknown cellular component",
  "gene_name": "SNF-related serine_threonine-protein kinase",
  "gene": "UniProtKB:Q9NRH2"
}